4-hydroxy-3-methoxy-5-polyprenylbenzoate decarboxylase activity [GO:0120539] (molecular function) Relationships: is_a GO:0016831; is part of ubiquinone biosynthetic process [GO:0006744] References: PMID:38295803, PMID:38425362 Sources: RHEA:81179 Definition: Catalysis of the reaction: a 4-hydroxy-3-methoxy-5-(all-trans-polyprenyl)benzoate + H+ = a 2-methoxy-6-(all-trans-polyprenyl)phenol + CO2.